{
  "gene_symbol": "HMOX1",
  "gene_name": "Heme oxygenase 1",
  "term_id": "GO:0006979",
  "gene": "UniProtKB:P09601",
  "term_label": "response to oxidative stress"
}